{
  "gene_symbol": "CD36",
  "gene": "UniProtKB:P16671",
  "term_id": "GO:0019915",
  "term_label": "lipid storage",
  "gene_name": "Platelet glycoprotein 4"
}